positive regulation of lysosomal membrane permeability [GO:0097214] (biological process) Relationships: is a type of regulation of lysosomal membrane permeability [GO:0097213]; is a type of positive regulation of membrane permeability [GO:1905710] Definition: Any process that increases the frequency, rate or extent of the passage or uptake of molecules by the lysosomal membrane. Also known as: positive regulation of lysosome membrane permeability References: PMID:20544854 Sources: GOC:yaf